{
  "gene": "UniProtKB:Q3KP44",
  "term_id": "UNKNOWN:0001",
  "term_label": "Unknown molecular function",
  "gene_name": "Ankyrin repeat domain-containing protein 55",
  "gene_symbol": "ANKRD55"
}